actomyosin contractile ring assembly actin filament organization [GO:2000689] (biological process) Subtypes: GO:0071519, actomyosin contractile ring assembly actin filament bundle convergence [GO:0071520], mitotic actomyosin contractile ring assembly actin filament organization [GO:1903479] Also known as: actin filament organisation of contractile ring assembly, actin filament organisation of cytokinesis, actomyosin contractile ring assembly, actin filament organization involved in cytokinetic actomyosin contractile ring assembly, actin filament organization of contractile ring assembly, actin filament organization of cytokinesis, actomyosin contractile ring assembly, actin filament organisation of constriction ring assembly, actin filament organisation of cytokinesis, actomyosin contractile ring formation, actin filament organisation of cytokinesis, actomyosin ring biosynthesis, actin filament organisation of cytokinesis, actomyosin ring formation, actin filament organisation of cytokinesis, contractile ring assembly, actin filament organization of constriction ring assembly, actin filament organization of cytokinesis, actomyosin contractile ring formation, actin filament organization of cytokinesis, actomyosin ring biosynthesis, actin filament organization of cytokinesis, actomyosin ring formation, actin filament organization of cytokinesis, contractile ring assembly, regulation of actin filament localization of constriction ring assembly, regulation of actin filament localization of contractile ring assembly, regulation of actin filament localization of cytokinesis, actomyosin contractile ring assembly, regulation of actin filament localization of cytokinesis, actomyosin contractile ring formation, regulation of actin filament localization of cytokinesis, actomyosin ring biosynthesis, regulation of actin filament localization of cytokinesis, actomyosin ring formation, regulation of actin filament localization of cytokinesis, contractile ring assembly Definition: An actin filament organization process that contributes to actomyosin contractile ring assembly during cytokinesis. Sources: GOC:mah Relationships: is a type of actin filament organization [GO:0007015]; is a type of cell cycle process [GO:0022402]; is part of actomyosin contractile ring assembly [GO:0000915]